{
  "gene_name": "Homeobox protein Hox-C10",
  "gene": "UniProtKB:Q9NYD6",
  "term_label": "regulation of transcription by RNA polymerase II",
  "gene_symbol": "HOXC10",
  "term_id": "GO:0006357"
}